MAD1 complex [GO:1990706] (cellular component) Definition: A protein complex involved in the assembly of the mitotic checkpoint complex that in turn inhibits the anaphase promoting complex/cyclosome (APC/C). Relationships: is a type of protein-containing complex [GO:0032991] References: PMID:22493223, PMID:22898774 Sources: GOC:bhm, intAct:EBI-10691224 Also known as: MAD1 homodimer